{
  "term_label": "visual perception",
  "gene_symbol": "CRYBA1",
  "term_id": "GO:0007601",
  "gene_name": "Beta-crystallin A3",
  "gene": "UniProtKB:P05813"
}